negative regulation of chanoclavine-I aldehyde biosynthetic process [GO:1900647] (biological process) Sources: GOC:TermGenie, GOC:di Also known as: down regulation of chanoclavine-I aldehyde anabolism, down regulation of chanoclavine-I aldehyde biosynthesis, down regulation of chanoclavine-I aldehyde biosynthetic process, down regulation of chanoclavine-I aldehyde formation, down regulation of chanoclavine-I aldehyde synthesis, down-regulation of chanoclavine-I aldehyde anabolism, down-regulation of chanoclavine-I aldehyde biosynthesis, down-regulation of chanoclavine-I aldehyde biosynthetic process, down-regulation of chanoclavine-I aldehyde formation, down-regulation of chanoclavine-I aldehyde synthesis, downregulation of chanoclavine-I aldehyde anabolism, downregulation of chanoclavine-I aldehyde biosynthesis, downregulation of chanoclavine-I aldehyde biosynthetic process, downregulation of chanoclavine-I aldehyde formation, downregulation of chanoclavine-I aldehyde synthesis, inhibition of chanoclavine-I aldehyde anabolism, inhibition of chanoclavine-I aldehyde biosynthesis, inhibition of chanoclavine-I aldehyde formation, inhibition of chanoclavine-I aldehyde synthesis, negative regulation of chanoclavine-I aldehyde anabolism, negative regulation of chanoclavine-I aldehyde biosynthesis, negative regulation of chanoclavine-I aldehyde formation, negative regulation of chanoclavine-I aldehyde synthesis, inhibition of chanoclavine-I aldehyde biosynthetic process Definition: Any process that stops, prevents or reduces the frequency, rate or extent of chanoclavine-I aldehyde biosynthetic process. Relationships: is a type of regulation of chanoclavine-I aldehyde biosynthetic process [GO:1900646]; is a type of negative regulation of ergot alkaloid biosynthetic process [GO:1900823]; negatively regulates GO:1900569